hypothalamus gonadotrophin-releasing hormone neuron differentiation [GO:0021886] (BP) Relationships: is a type of hypothalamus cell differentiation [GO:0021979] Also known as: hypothalamus gonadotropin-releasing hormone neuron differentiation References: PMID:12626695 Sources: GOC:cls, GOC:dgh, GOC:dph, GOC:jid, GO_REF:0000021 Definition: The process in which a relatively unspecialized cell acquires specialized features of a neuron located in the hypothalamus. These neurons release gonadotrophin-releasing hormone as a neural transmitter.